{
  "gene": "UniProtKB:A0AUZ9",
  "gene_symbol": "KANSL1L",
  "gene_name": "KAT8 regulatory NSL complex subunit 1-like protein",
  "term_id": "UNKNOWN:0002",
  "term_label": "Unknown biological process"
}